{
  "term_id": "GO:0017116",
  "gene_name": "DNA replication licensing factor MCM3",
  "gene_symbol": "MCM3",
  "gene": "UniProtKB:P25205",
  "term_label": "single-stranded DNA helicase activity"
}